{
  "term_label": "cysteine-type deubiquitinase activity",
  "gene_name": "Ubiquitin carboxyl-terminal hydrolase 48",
  "term_id": "GO:0004843",
  "gene": "UniProtKB:Q86UV5",
  "gene_symbol": "USP48"
}